astral microtubule organization [GO:0030953] (biological process) Subtypes: astral microtubule nucleation [GO:0030954], astral microtubule depolymerization [GO:0060172] Definition: A process that is carried out at the cellular level which results in the assembly, arrangement of constituent parts, or disassembly of astral microtubules, any of the spindle microtubules that radiate in all directions from the spindle poles. Also known as: astral microtubule organisation, astral microtubule organization and biogenesis Sources: GOC:mah Relationships: is a type of spindle organization [GO:0007051]; is a type of cytoplasmic microtubule organization [GO:0031122]